{
  "term_label": "transmembrane transporter binding",
  "term_id": "GO:0044325",
  "gene": "UniProtKB:A6NFQ2",
  "gene_name": "TRPM8 channel-associated factor 2",
  "gene_symbol": "TCAF2"
}